{
  "gene_name": "DNA helicase MCM8",
  "term_label": "double-strand break repair via homologous recombination",
  "gene_symbol": "MCM8",
  "gene": "UniProtKB:Q9UJA3",
  "term_id": "GO:0000724"
}